thiamine diphosphate catabolic process [GO:0042358] (biological process) Definition: The chemical reactions and pathways resulting in the breakdown of thiamine diphosphate, a derivative of thiamine (vitamin B1) which acts as a coenzyme in a range of processes including the Krebs cycle. Sources: GOC:jl, ISBN:0198506732 Also known as: TPP catabolic process, TPP catabolism, thiamin diphosphate breakdown, thiamin diphosphate catabolic process, thiamin diphosphate catabolism, thiamin diphosphate degradation, thiamin pyrophosphate catabolic process, thiamin pyrophosphate catabolism, thiamine diphosphate catabolism, thiamine pyrophosphate catabolic process, thiamine pyrophosphate catabolism Relationships: is a type of thiamine diphosphate metabolic process [GO:0042357]; is a type of GO:0042725; is a type of organophosphate catabolic process [GO:0046434]